{
  "term_label": "calcium ion binding",
  "gene_symbol": "ITPR1",
  "term_id": "GO:0005509",
  "gene": "UniProtKB:Q14643",
  "gene_name": "Inositol 1,4,5-trisphosphate receptor type 1"
}